{
  "term_id": "GO:0048013",
  "gene": "UniProtKB:P16333",
  "gene_symbol": "NCK1",
  "gene_name": "Cytoplasmic protein NCK1",
  "term_label": "ephrin receptor signaling pathway"
}